positive regulation of IP-10 production [GO:0071660] (biological process) Sources: GOC:mah Definition: Any process that activates or increases the frequency, rate, or extent of production of IP-10. Relationships: is a type of positive regulation of chemokine production [GO:0032722]; is a type of GO:0071658; RO_0002213 IP-10 production [GO:0071612] Also known as: positive regulation of CXCL10 production, positive regulation of chemokine (C-C motif) ligand 10 production